{
  "term_id": "GO:0000981",
  "gene_name": "Myogenic factor 6",
  "gene": "UniProtKB:P23409",
  "gene_symbol": "MYF6",
  "term_label": "DNA-binding transcription factor activity, RNA polymerase II-specific"
}